{
  "gene": "UniProtKB:Q07108",
  "term_label": "Unknown biological process",
  "gene_symbol": "CD69",
  "term_id": "UNKNOWN:0002",
  "gene_name": "Early activation antigen CD69"
}